{
  "gene": "UniProtKB:Q9BSG5",
  "term_id": "GO:1902444",
  "term_label": "riboflavin binding",
  "gene_symbol": "RTBDN",
  "gene_name": "Retbindin"
}